astrocyte development [GO:0014002] (biological process) Also known as: astrocyte cell development Relationships: is a type of glial cell development [GO:0021782]; is part of astrocyte differentiation [GO:0048708] Definition: The process aimed at the progression of an astrocyte over time, from initial commitment of the cell to a specific fate, to the fully functional differentiated cell. An astrocyte is the most abundant type of glial cell. Astrocytes provide support for neurons and regulate the environment in which they function. Subtypes: forebrain astrocyte development [GO:0021897] Sources: GOC:dgh, GOC:ef